{
  "gene_name": "Diphosphoinositol polyphosphate phosphohydrolase 3-beta",
  "term_label": "adenosine 5'-(hexahydrogen pentaphosphate) catabolic process",
  "term_id": "GO:1901911",
  "gene": "UniProtKB:Q96G61",
  "gene_symbol": "NUDT11"
}